{
  "gene": "UniProtKB:Q9UP38",
  "term_id": "GO:0042813",
  "gene_symbol": "FZD1",
  "term_label": "Wnt receptor activity",
  "gene_name": "Frizzled-1"
}